{
  "gene_name": "Endogenous retrovirus group K member 18 Pol protein",
  "term_label": "RNA stem-loop binding",
  "gene": "UniProtKB:Q9QC07",
  "term_id": "GO:0035613",
  "gene_symbol": "ERVK-18"
}